alpha-zeacarotene catabolic process [GO:1901820] (biological process) References: PMID:6060456 Sources: GOC:TermGenie, GOC:yaf, UniPathway:UPA00804 Relationships: is a type of carotenoid catabolic process [GO:0016118]; is a type of carotene catabolic process [GO:0016121] Also known as: alpha-zeacarotene breakdown, alpha-zeacarotene catabolism, alpha-zeacarotene degradation Definition: The chemical reactions and pathways resulting in the breakdown of alpha-zeacarotene.